{
  "gene_name": "Adenylate kinase 8",
  "gene_symbol": "AK8",
  "term_id": "GO:0005737",
  "gene": "UniProtKB:Q96MA6",
  "term_label": "cytoplasm"
}